{
  "term_id": "GO:0070588",
  "gene_symbol": "ATP2A3",
  "term_label": "calcium ion transmembrane transport",
  "gene_name": "Sarcoplasmic_endoplasmic reticulum calcium ATPase 3",
  "gene": "UniProtKB:Q93084"
}